beta-N-acetylglucosaminidase activity [GO:0016231] (molecular function) Definition: Catalysis of the hydrolysis of terminal non-reducing N-acetyl-D-glucosamine residues in N-acetyl-beta-D-glucosaminides. Relationships: is a type of beta-N-acetylhexosaminidase activity [GO:0004563] References: PMID:29143882, PMID:37590576